{
  "gene_name": "KIR2DL1 protein",
  "term_label": "transmembrane signaling receptor activity",
  "gene_symbol": "KIR2DL1",
  "term_id": "GO:0004888",
  "gene": "UniProtKB:A0A5K1VDZ0"
}